{
  "term_id": "GO:0005952",
  "gene": "UniProtKB:P13861",
  "term_label": "cAMP-dependent protein kinase complex",
  "gene_symbol": "PRKAR2A",
  "gene_name": "cAMP-dependent protein kinase type II-alpha regulatory subunit"
}